formaldehyde assimilation via ribulose monophosphate cycle [GO:0019647] (BP) Definition: The pathway in which formaldehyde is used as a carbon source in the ribulose monophosphate cycle. Methanotrophic bacteria produce formaldehyde from the oxidation of methane and methanol, and then assimilate it via the ribulose monophosphate cycle to form intermediates of the central metabolic routes that are subsequently used for biosynthesis of cell material. Three molecules of formaldehyde are assimilated, forming a three-carbon intermediate of central metabolism; in this pathway, all cellular carbon is assimilated at the oxidation level of formaldehyde. Relationships: is a type of formaldehyde assimilation [GO:0019649] Also known as: ribulose monophosphate cycle, formaldehyde assimilation via RuMP cycle Sources: MetaCyc:PWY-1861